{
  "gene_name": "Protein FAM53A",
  "gene": "UniProtKB:Q6NSI3",
  "term_id": "GO:0006606",
  "term_label": "protein import into nucleus",
  "gene_symbol": "FAM53A"
}